{
  "term_label": "cytosol",
  "gene": "UniProtKB:Q13283",
  "term_id": "GO:0005829",
  "gene_name": "Ras GTPase-activating protein-binding protein 1",
  "gene_symbol": "G3BP1"
}